{
  "gene": "UniProtKB:Q96PJ5",
  "gene_name": "Fc receptor-like protein 4",
  "gene_symbol": "FCRL4",
  "term_label": "immune response",
  "term_id": "GO:0006955"
}